{
  "gene_name": "Mitogen-activated protein kinase kinase kinase 5",
  "term_label": "JNK cascade",
  "gene": "UniProtKB:Q99683",
  "term_id": "GO:0007254",
  "gene_symbol": "MAP3K5"
}